lysine biosynthetic process via diaminopimelate and N-succinyl-2-amino-6-ketopimelate [GO:0033359] (biological process) Definition: The chemical reactions and pathways resulting in the formation of lysine, via the intermediates diaminopimelate and N-succinyl-2-amino-6-ketopimelate; in this pathway tetrahydrodipicolinate is converted to meso-diaminopimelate in four enzymatic steps. Sources: GOC:mah, MetaCyc:DAPLYSINESYN-PWY Also known as: lysine anabolism via diaminopimelate and N-succinyl-2-amino-6-ketopimelate, lysine biosynthesis via diaminopimelic acid and N-succinyl-2-amino-6-ketopimelate, lysine biosynthetic process via diaminopimelic acid and N-succinyl-2-amino-6-ketopimelate, lysine formation via diaminopimelate and N-succinyl-2-amino-6-ketopimelate, lysine synthesis via diaminopimelate and N-succinyl-2-amino-6-ketopimelate Relationships: is a type of lysine biosynthetic process via diaminopimelate [GO:0009089]